farnesol dehydrogenase activity [GO:0047886] (molecular function) Also known as: 2-trans,6-trans-farnesol:NADP+ 1-oxidoreductase activity, NADP-farnesol dehydrogenase activity, farnesol (nicotinamide adenine dinucleotide phosphate) dehydrogenase activity Relationships: is a type of oxidoreductase activity, acting on the CH-OH group of donors, NAD or NADP as acceptor [GO:0016616] Sources: EC:1.1.1.216, RHEA:14697 Definition: Catalysis of the reaction: 2-trans,6-trans-farnesol + NADP+ = 2-trans,6-trans-farnesal + H+ + NADPH.